{
  "term_label": "neuropeptide signaling pathway",
  "term_id": "GO:0007218",
  "gene": "UniProtKB:P30874",
  "gene_name": "Somatostatin receptor type 2",
  "gene_symbol": "SSTR2"
}